{
  "term_label": "nucleus",
  "gene_name": "DNA dC-dU-editing enzyme APOBEC-3B",
  "term_id": "GO:0005634",
  "gene_symbol": "APOBEC3B",
  "gene": "UniProtKB:Q9UH17"
}